{
  "gene_name": "Eukaryotic translation initiation factor 2 subunit 2",
  "gene": "UniProtKB:P20042",
  "term_label": "eukaryotic translation initiation factor 2 complex",
  "gene_symbol": "EIF2S2",
  "term_id": "GO:0005850"
}